notum development [GO:0007477] (biological process) Definition: The process whose specific outcome is the progression of the dorsal part of the body over time, from its formation to the mature structure. Relationships: is a type of anatomical structure development [GO:0048856]; BFO_0000050 GO:0035220 Sources: GOC:jid